9,9'-di-cis-zeta-carotene desaturation to 7,9,7',9'-tetra-cis-lycopene [GO:0052889] (biological process) Definition: The series of reactions in which 9,9'-di-cis-zeta-carotene is desaturated to 7,9,9'-tri-cis-neurosporene, and then 7,9,7',9'-tetra-cis-lycopene. The overall reaction for this process is: 9,9'-di-cis-zeta-carotene + 2 quinone = 2 quinol + 7,9,7',9'-tetra-cis-lycopene. Sources: MetaCyc:PWY-6475 Also known as: 7,9,7',9'-tetra-cis-lycopene biosynthesis from 9,9'-di-cis-zeta-carotene, 9,9'-di-cis-zeta-carotene catabolism to 7,9,7',9'-tetra-cis-lycopene Relationships: is a type of GO:0016119; has part GO:0016719